{
  "term_id": "GO:0006094",
  "gene_symbol": "GPI",
  "gene_name": "Glucose-6-phosphate isomerase",
  "gene": "UniProtKB:P06744",
  "term_label": "gluconeogenesis"
}